{
  "term_id": "GO:0060326",
  "term_label": "cell chemotaxis",
  "gene": "UniProtKB:P32246",
  "gene_name": "C-C chemokine receptor type 1",
  "gene_symbol": "CCR1"
}